{
  "gene": "UniProtKB:P07988",
  "gene_name": "Pulmonary surfactant-associated protein B",
  "term_id": "GO:0005615",
  "gene_symbol": "SFTPB",
  "term_label": "extracellular space"
}